type I site-specific deoxyribonuclease complex [GO:0019812] (cellular component) Definition: A multisubunit complex composed of two copies of a restriction (R) subunit, two copies of a methylation (M) subunit, and one copy of a specificity (S) subunit. This complex recognizes specific short DNA sequences (through the S subunit), and binds to them. If the recognition site is hemimethylated, the complex acts as a methyltransferase which modifies the recognition site, using S-adenosylmethionine as the methyl donor. Only the M and S subunits are required for this reaction. If the complex binds to an unmethylated recognition site, then the complex translocates the DNA bidirectionally in an ATP-dependent manner. When the translocation is stalled by impact with another complex or unusual DNA structure, the enzyme functions as an endonuclease and cleavage of the DNA will occur, hundreds or thousands of base pairs away from the recognition site. These DNA restriction systems are used by bacteria to defend against phage and other foreign DNA that may enter a cell. References: PMID:12654995, PMID:15788748 Also known as: type I restriction enzyme complex Relationships: is a type of endodeoxyribonuclease complex [GO:1905347]; is part of GO:0005737